regulation of transport [GO:0051049] (biological process) Definition: Any process that modulates the frequency, rate or extent of the directed movement of substances (such as macromolecules, small molecules, ions) into, out of or within a cell, or between cells, by means of some agent such as a transporter or pore. Sources: GOC:ai Relationships: is a type of regulation of localization [GO:0032879]; regulates transport [GO:0006810] Subtypes: regulation of phosphate transport [GO:0010966], GO:0032239, regulation of lipid transport [GO:0032368], regulation of intracellular transport [GO:0032386], GO:0032890, regulation of transmembrane transport [GO:0034762], regulation of monoatomic ion transport [GO:0043269], regulation of secretion [GO:0051046], GO:0051050, negative regulation of transport [GO:0051051], regulation of protein transport [GO:0051223], regulation of neurotransmitter transport [GO:0051588], GO:0051621, GO:0051626, GO:0051952, regulation of vesicle-mediated transport [GO:0060627], regulation of peptide transport [GO:0090087], GO:0150111, regulation of transport across blood-brain barrier [GO:0150200], GO:1900285, regulation of galactotriose transport [GO:1900291], regulation of heptasaccharide transport [GO:1900294], regulation of hexasaccharide transport [GO:1900297], regulation of laminaritriose transport [GO:1900303], GO:1900321, regulation of maltotriulose transport [GO:1900324], GO:1900327, regulation of nigerotriose transport [GO:1900357], GO:1900360, GO:1901028, regulation of maltose transport [GO:1902343], regulation of synaptic vesicle transport [GO:1902803], GO:1902908, GO:1903421, GO:2000012, regulation of renal water transport [GO:2001151]